{
  "gene_symbol": "PTPRT",
  "term_label": "signal transduction",
  "gene": "UniProtKB:O14522",
  "gene_name": "Receptor-type tyrosine-protein phosphatase T",
  "term_id": "GO:0007165"
}